{
  "gene_name": "FUN14 domain-containing protein 1",
  "term_label": "autophagy of mitochondrion",
  "gene_symbol": "FUNDC1",
  "term_id": "GO:0000422",
  "gene": "UniProtKB:Q8IVP5"
}